{
  "gene_symbol": "IGF2BP2",
  "gene": "UniProtKB:Q9Y6M1",
  "gene_name": "Insulin-like growth factor 2 mRNA-binding protein 2",
  "term_label": "nucleus",
  "term_id": "GO:0005634"
}